detection of hypoxia [GO:0070483] (biological process) Sources: GOC:BHF, GOC:mah Subtypes: detection of reduced oxygen by chemoreceptor signaling [GO:0003020] Definition: The series of events in which a stimulus indicating lowered oxygen tension is received by a cell and converted into a molecular signal. Hypoxia, defined as a decline in O2 levels below normoxic levels of 20.8 - 20.95%, results in metabolic adaptation at both the cellular and organismal level. Relationships: is a type of response to hypoxia [GO:0001666]; is a type of GO:0003032 Also known as: detection of reduced oxygen levels